{
  "gene": "UniProtKB:P11441",
  "term_label": "tail-anchored membrane protein insertion into ER membrane",
  "gene_name": "Ubiquitin-like protein 4A",
  "term_id": "GO:0071816",
  "gene_symbol": "UBL4A"
}